positive regulation of centrosome cycle [GO:0046607] (biological process) Sources: GOC:ai Also known as: up regulation of centrosome cycle, up-regulation of centrosome cycle, upregulation of centrosome cycle, activation of centrosome cycle, stimulation of centrosome cycle Definition: Any process that activates or increases the frequency, rate or extent of the centrosome cycle. Relationships: is a type of regulation of centrosome cycle [GO:0046605]; is a type of positive regulation of cytoskeleton organization [GO:0051495]; is a type of GO:0090068; positively regulates centrosome cycle [GO:0007098]